{
  "gene_name": "Unconventional myosin-Ie",
  "gene": "UniProtKB:Q12965",
  "gene_symbol": "MYO1E",
  "term_id": "GO:0015629",
  "term_label": "actin cytoskeleton"
}